{
  "gene_symbol": "SMIM43",
  "gene": "UniProtKB:Q4W5P6",
  "term_label": "Unknown cellular component",
  "term_id": "UNKNOWN:0003",
  "gene_name": "Small integral membrane protein 43"
}